purine deoxyribonucleoside interconversion [GO:0019688] (biological process) Relationships: is a type of purine nucleoside interconversion [GO:0019686]; is a type of GO:0046122 Sources: GOC:mah, ISBN:0306444747, ISBN:0471394831 Definition: The chemical reactions and pathways by which a purine deoxyribonucleoside is synthesized from another purine deoxyribonucleoside.